negative regulation of white fat cell differentiation [GO:0160275] (biological process) Relationships: is a type of negative regulation of fat cell differentiation [GO:0045599]; negatively regulates white fat cell differentiation [GO:0050872] References: PMID:24703692 Definition: Any process that stops, prevents or reduces the frequency, rate or extent of white fat cell differentiation.